positive regulation of heart contraction [GO:0045823] (biological process) Definition: Any process that activates or increases the frequency, rate or extent of heart contraction. Sources: GOC:go_curators Also known as: positive regulation of cardiac contraction, up regulation of heart contraction, up-regulation of heart contraction, upregulation of heart contraction, activation of heart contraction, stimulation of heart contraction Relationships: is a type of regulation of heart contraction [GO:0008016]; is a type of positive regulation of blood circulation [GO:1903524]; positively regulates heart contraction [GO:0060047] Subtypes: positive regulation of the force of heart contraction by chemical signal [GO:0003099], positive regulation of heart rate [GO:0010460], positive regulation of cardiac muscle contraction [GO:0060452]